{
  "term_id": "GO:0031410",
  "gene_symbol": "AMOTL2",
  "gene_name": "Angiomotin-like protein 2",
  "term_label": "cytoplasmic vesicle",
  "gene": "UniProtKB:Q9Y2J4"
}